dimethylmalate dehydrogenase activity [GO:0047867] (molecular function) Also known as: (R)-3,3-dimethylmalate:NAD+ oxidoreductase (decarboxylating), beta,beta-dimethylmalate dehydrogenase activity Sources: EC:1.1.1.84, RHEA:13321 Relationships: is_a oxidoreductase activity, acting on the CH-OH group of donors, NAD or NADP as acceptor [GO:0016616] Definition: Catalysis of the reaction: (R)-3,3-dimethylmalate + NAD+ = 3-methyl-2-oxobutanoate + CO2 + NADH.